{
  "gene_name": "Homeobox protein Hox-B3",
  "gene": "UniProtKB:P14651",
  "gene_symbol": "HOXB3",
  "term_id": "GO:0009952",
  "term_label": "anterior/posterior pattern specification"
}